{
  "term_id": "GO:0034486",
  "term_label": "vacuolar transmembrane transport",
  "gene_symbol": "SLC46A3",
  "gene": "UniProtKB:Q7Z3Q1",
  "gene_name": "Lysosomal proton-coupled steroid conjugate and bile acid symporter SLC46A3"
}